type 1D serotonin receptor binding [GO:0031823] (molecular function) Also known as: 5-hydroxytryptamine 1D receptor binding, type 1D serotonin receptor ligand Definition: Binding to a type 1D serotonin receptor. Sources: GOC:mah, GOC:nln Relationships: is a type of G protein-coupled serotonin receptor binding [GO:0031821]